apoptotic chromosome condensation [GO:0030263] (biological process) Definition: The compaction of chromatin during apoptosis. Also known as: pyknosis Sources: GOC:mah Relationships: is a type of GO:0030261; is part of apoptotic nuclear changes [GO:0030262]